{
  "gene_name": "Meiotic recombination protein REC114",
  "gene_symbol": "REC114",
  "term_label": "Unknown biological process",
  "term_id": "UNKNOWN:0002",
  "gene": "UniProtKB:Q7Z4M0"
}